biological process involved in interspecies interaction between organisms [GO:0044419] (BP) Also known as: interaction with another species, interspecies interaction, interspecies interaction between organisms, interspecies interaction with other organisms Relationships: is a type of biological_process [GO:0008150] Definition: Any process evolved to enable an interaction with an organism of a different species. Subtypes: modulation of process of another organism [GO:0035821], formation of structure involved in a symbiotic process [GO:0044111], biological process involved in symbiotic interaction [GO:0044403], GO:0051707, GO:0140106, disruption of anatomical structure in another organism [GO:0141060] Sources: GOC:cc